{
  "term_id": "GO:0032281",
  "gene": "UniProtKB:Q9ULK0",
  "term_label": "AMPA glutamate receptor complex",
  "gene_symbol": "GRID1",
  "gene_name": "Glutamate receptor ionotropic, delta-1"
}